{
  "gene_symbol": "HDLBP",
  "term_label": "Unknown cellular component",
  "gene": "UniProtKB:Q00341",
  "gene_name": "Vigilin",
  "term_id": "UNKNOWN:0003"
}